cytidine kinase activity [GO:0043771] (molecular function) References: PMID:211379 Sources: RHEA:24674 Definition: Catalysis of the reaction: ATP + cytidine = ADP + CMP. Also known as: uridine-cytidine kinase activity Relationships: is a type of nucleoside kinase activity [GO:0019206]; is part of CMP biosynthetic process [GO:0009224]